{
  "term_id": "GO:0070989",
  "gene": "UniProtKB:P08684",
  "term_label": "oxidative demethylation",
  "gene_symbol": "CYP3A4",
  "gene_name": "Cytochrome P450 3A4"
}